protein-glutamic acid ligase activity [GO:0070739] (molecular function) Definition: Catalysis of the posttranslational transfer of one or more glutamate residues to a specific residue on a target protein. Also known as: protein glutamylase activity, protein-glutamate ligase activity Relationships: is a type of acid-amino acid ligase activity [GO:0016881]; is a type of catalytic activity, acting on a protein [GO:0140096] References: PMID:19524510 Sources: GOC:mah Subtypes: ribosomal S6-glutamic acid ligase activity [GO:0018169], GO:0070740, protein-glutamic acid ligase activity, initiating [GO:0106437], GO:0106438